{
  "term_label": "odorant binding",
  "gene_name": "Olfactory receptor 5M3",
  "term_id": "GO:0005549",
  "gene_symbol": "OR5M3",
  "gene": "UniProtKB:Q8NGP4"
}